{
  "gene": "UniProtKB:Q6ZMH5",
  "term_id": "GO:0005385",
  "gene_symbol": "SLC39A5",
  "term_label": "zinc ion transmembrane transporter activity",
  "gene_name": "Zinc transporter ZIP5"
}